negative regulation of 'de novo' NAD biosynthetic process from L-tryptophan [GO:1905013] (biological process) Relationships: is a type of negative regulation of amino acid metabolic process [GO:0045763]; is a type of negative regulation of purine nucleotide biosynthetic process [GO:1900372]; is a type of negative regulation of NAD metabolic process [GO:1902689]; is a type of regulation of 'de novo' NAD biosynthetic process from L-tryptophan [GO:1905012]; negatively regulates 'de novo' NAD+ biosynthetic process from L-tryptophan [GO:0034354] References: PMID:12140278, PMID:19843166 Sources: GOC:PARL, GOC:TermGenie, GOC:bf, GO_REF:0000058 Also known as: negative regulation of 'de novo' NAD biosynthetic process from tryptophan, down regulation of 'de novo' NAD biosynthetic process from tryptophan, down-regulation of 'de novo' NAD biosynthetic process from tryptophan, downregulation of 'de novo' NAD biosynthetic process from tryptophan, inhibition of 'de novo' NAD biosynthetic process from tryptophan, down regulation of de novo NAD biosynthetic process from tryptophan, down-regulation of de novo NAD biosynthetic process from tryptophan, downregulation of de novo NAD biosynthetic process from tryptophan, inhibition of de novo NAD biosynthetic process from tryptophan, negative regulation of de novo NAD biosynthetic process from tryptophan Definition: Any process that stops, prevents or reduces the frequency, rate or extent of 'de novo' NAD biosynthetic process from L-tryptophan.